{
  "gene_name": "RalA-binding protein 1",
  "term_id": "GO:0005096",
  "term_label": "GTPase activator activity",
  "gene": "UniProtKB:Q15311",
  "gene_symbol": "RALBP1"
}